ribonucleotide binding [GO:0032553] (molecular function) Definition: Binding to a ribonucleotide, any compound consisting of a ribonucleoside that is esterified with (ortho)phosphate or an oligophosphate at any hydroxyl group on the ribose moiety. Sources: GOC:mah Relationships: is a type of nucleotide binding [GO:0000166]; is a type of carbohydrate derivative binding [GO:0097367] Subtypes: GO:0010181, purine ribonucleotide binding [GO:0032555], pyrimidine ribonucleotide binding [GO:0032557], GO:0120233